{
  "gene": "UniProtKB:Q92567",
  "gene_symbol": "FAM168A",
  "term_id": "UNKNOWN:0001",
  "term_label": "Unknown molecular function",
  "gene_name": "Protein FAM168A"
}